{
  "term_label": "structural constituent of ribosome",
  "gene_symbol": "MRPS22",
  "gene": "UniProtKB:P82650",
  "term_id": "GO:0003735",
  "gene_name": "Small ribosomal subunit protein mS22"
}